regulation of chanoclavine-I aldehyde biosynthetic process [GO:1900646] (biological process) Sources: GOC:TermGenie, GOC:di Also known as: regulation of chanoclavine-I aldehyde anabolism, regulation of chanoclavine-I aldehyde biosynthesis, regulation of chanoclavine-I aldehyde formation, regulation of chanoclavine-I aldehyde synthesis Definition: Any process that modulates the frequency, rate or extent of chanoclavine-I aldehyde biosynthetic process. Subtypes: negative regulation of chanoclavine-I aldehyde biosynthetic process [GO:1900647], positive regulation of chanoclavine-I aldehyde biosynthetic process [GO:1900648] Relationships: is a type of regulation of ergot alkaloid biosynthetic process [GO:1900822]; regulates chanoclavine-I aldehyde biosynthetic process [GO:1900569]